vasodilation involved in acute inflammatory response [GO:0002527] (biological process) Also known as: vasodilation during acute inflammatory response Definition: An increase in the internal diameter of blood vessels, especially arterioles or capillaries, usually resulting in a decrease in blood pressure contributing to an acute inflammatory response. Relationships: is a type of vasodilation [GO:0042311]; is part of acute inflammatory response [GO:0002526] Sources: GOC:jal